{
  "gene_symbol": "EIF3A",
  "term_id": "GO:0003729",
  "gene": "UniProtKB:Q14152",
  "term_label": "mRNA binding",
  "gene_name": "Eukaryotic translation initiation factor 3 subunit A"
}